{
  "gene_symbol": "QTRT1",
  "gene": "UniProtKB:Q9BXR0",
  "gene_name": "Queuine tRNA-ribosyltransferase catalytic subunit 1",
  "term_id": "UNKNOWN:0003",
  "term_label": "Unknown cellular component"
}